{
  "term_id": "GO:0009986",
  "gene_symbol": "GPC1",
  "term_label": "cell surface",
  "gene": "UniProtKB:P35052",
  "gene_name": "Glypican-1"
}